{
  "term_id": "GO:0042274",
  "gene_symbol": "IMP3",
  "gene": "UniProtKB:Q9NV31",
  "term_label": "ribosomal small subunit biogenesis",
  "gene_name": "U3 small nucleolar ribonucleoprotein protein IMP3"
}